endogenous antibiotic catabolic process [GO:0042741] (biological process) Definition: The chemical reactions and pathways resulting in the breakdown of an antibiotic that has originated internally within the cell or organism. Sources: GOC:jl Also known as: endogenous antibiotic breakdown, endogenous antibiotic catabolism, endogenous antibiotic degradation Relationships: is_a antibiotic catabolic process [GO:0017001]